{
  "gene": "UniProtKB:Q9NZ94",
  "gene_symbol": "NLGN3",
  "term_id": "GO:0009986",
  "term_label": "cell surface",
  "gene_name": "Neuroligin-3"
}